{
  "gene_name": "Forkhead box protein O1",
  "gene": "UniProtKB:Q12778",
  "term_label": "positive regulation of gluconeogenesis",
  "gene_symbol": "FOXO1",
  "term_id": "GO:0045722"
}